negative regulation of maintenance of sister chromatid cohesion [GO:0034092] (biological process) Definition: Any process that decreases the extent to which the association between sister chromatids of a replicated chromosome is maintained. Sources: GOC:mah, GOC:vw Relationships: is a type of regulation of maintenance of sister chromatid cohesion [GO:0034091]; is a type of negative regulation of sister chromatid cohesion [GO:0045875]; RO_0002212 maintenance of sister chromatid cohesion [GO:0034086] Subtypes: negative regulation of maintenance of meiotic sister chromatid cohesion [GO:0034095], GO:0034183